{
  "gene_name": "Scavenger receptor cysteine-rich domain-containing protein SCART1",
  "gene_symbol": "SCART1",
  "gene": "UniProtKB:Q4G0T1",
  "term_label": "plasma membrane",
  "term_id": "GO:0005886"
}